{
  "gene_symbol": "JAKMIP3",
  "gene_name": "Janus kinase and microtubule-interacting protein 3",
  "term_label": "Unknown cellular component",
  "term_id": "UNKNOWN:0003",
  "gene": "UniProtKB:Q5VZ66"
}